actin-mediated cell contraction [GO:0070252] (biological process) Relationships: is a type of actin filament-based movement [GO:0030048] Subtypes: apical constriction [GO:0003383], actin-myosin filament sliding [GO:0033275], GO:0060327, hepatic stellate cell contraction [GO:0061872], cardiac muscle cell contraction [GO:0086003], cochlear outer hair cell electromotile response [GO:0099129], myofibroblast contraction [GO:1990764] Definition: The actin filament-based process in which cytoplasmic actin filaments slide past one another resulting in contraction of all or part of the cell body. Sources: GOC:mah